{
  "term_label": "myosin heavy chain binding",
  "gene": "UniProtKB:O14950",
  "gene_name": "Myosin regulatory light chain 12B",
  "term_id": "GO:0032036",
  "gene_symbol": "MYL12B"
}